{
  "gene_name": "Paired box protein Pax-2",
  "term_label": "Unknown cellular component",
  "gene_symbol": "PAX2",
  "gene": "UniProtKB:Q02962",
  "term_id": "UNKNOWN:0003"
}